{
  "gene_symbol": "DNAH14",
  "term_label": "9+2 motile cilium",
  "term_id": "GO:0097729",
  "gene_name": "Dynein axonemal heavy chain 14",
  "gene": "UniProtKB:Q0VDD8"
}